{
  "gene": "UniProtKB:H3BU10",
  "gene_symbol": "MGC35212",
  "term_label": "Unknown molecular function",
  "gene_name": "Cell division control protein 24 OB domain-containing protein",
  "term_id": "UNKNOWN:0001"
}